MyD88-dependent toll-like receptor 2 signaling pathway [GO:0035661] (biological process) Also known as: MyD88-dependent TLR2 signaling pathway, MyD88-dependent toll-like receptor 2 signalling pathway Relationships: is a type of MyD88-dependent toll-like receptor signaling pathway [GO:0002755]; is a type of GO:0034134 References: PMID:20385024 Sources: GOC:BHF Definition: The series of molecular signals initiated by a ligand binding to a toll-like 2 receptor where the MyD88 adaptor molecule mediates transduction of the signal. Toll-like 2 receptors are pattern recognition receptors that bind microbial pattern motifs to initiate an innate immune response.